{
  "gene": "UniProtKB:Q96GX9",
  "term_id": "GO:0046570",
  "term_label": "methylthioribulose 1-phosphate dehydratase activity",
  "gene_symbol": "APIP",
  "gene_name": "Methylthioribulose-1-phosphate dehydratase"
}